acquisition of desiccation tolerance [GO:0097439] (biological process) Relationships: is a type of GO:0022611 Sources: GOC:PO_curators Definition: The process in which tolerance to severe drying is acquired, before entering into a dry, either dormant or quiescent state. Subtypes: GO:0048700